purine nucleobase catabolic process [GO:0006145] (biological process) Relationships: is a type of purine nucleobase metabolic process [GO:0006144]; is a type of nucleobase catabolic process [GO:0046113]; is a type of GO:0072523 Sources: GOC:go_curators Subtypes: adenine catabolic process [GO:0006146], guanine catabolic process [GO:0006147], hypoxanthine catabolic process [GO:0009114], xanthine catabolic process [GO:0009115], anaerobic purine nucleobase catabolic process [GO:0019653] Definition: The chemical reactions and pathways resulting in the breakdown of purine nucleobases, one of the two classes of nitrogen-containing ring compounds found in DNA and RNA, which include adenine and guanine. Also known as: purine base breakdown, purine base catabolic process, purine base catabolism, purine base degradation